sodium-independent leukotriene transport [GO:0071719] (biological process) Relationships: is a type of leukotriene transport [GO:0071716]; is a type of sodium-independent icosanoid transport [GO:0071718] Sources: GOC:mah Definition: The directed, sodium-independent, movement of leukotrienes into, out of or within a cell, or between cells, by means of some agent such as a transporter or pore. Leukotrienes are linear C20 endogenous metabolites of arachidonic acid (icosa-5,8,11,14-tetraenoic acid) containing a terminal carboxy function and four or more double bonds (three or more of which are conjugated) as well as other functional groups.